visceral muscle development [GO:0007522] (biological process) Subtypes: larval visceral muscle development [GO:0007523], GO:0007524 Sources: GOC:go_curators Definition: The process whose specific outcome is the progression of the visceral muscle over time, from its formation to the mature structure. Relationships: is a type of muscle organ development [GO:0007517]